{
  "gene_symbol": "ZNF250",
  "gene_name": "Zinc finger protein 250",
  "gene": "UniProtKB:P15622",
  "term_label": "nucleus",
  "term_id": "GO:0005634"
}